{
  "gene_name": "Calpain-9",
  "term_id": "GO:0006508",
  "term_label": "proteolysis",
  "gene_symbol": "CAPN9",
  "gene": "UniProtKB:O14815"
}